regulation of excitatory postsynaptic membrane potential involved in skeletal muscle contraction [GO:0014853] (biological process) Also known as: regulation of excitatory post-synaptic membrane potential involved in skeletal muscle contraction Relationships: is a type of modulation of excitatory postsynaptic potential [GO:0098815]; is part of GO:0003009; BFO_0000050 regulation of skeletal muscle contraction by neural stimulation via neuromuscular junction [GO:0014852] Sources: GOC:ef, GOC:mtg_muscle Definition: Any process, involved in skeletal muscle contraction, that modulates the establishment or extent of the excitatory postsynaptic potential (EPSP). Excitatory postsynaptic potential (EPSP) is a temporary increase in postsynaptic potential due to the flow of positively charged ions into the postsynaptic cell. The flow of ions that causes an EPSP is an excitatory postsynaptic current (EPSC) and makes it easier for the neuron to fire an action potential.